{
  "term_id": "GO:0019957",
  "gene_name": "Atypical chemokine receptor 4",
  "gene_symbol": "ACKR4",
  "term_label": "C-C chemokine binding",
  "gene": "UniProtKB:Q9NPB9"
}